{
  "term_label": "profilin binding",
  "gene_name": "Protein enabled homolog",
  "term_id": "GO:0005522",
  "gene_symbol": "ENAH",
  "gene": "UniProtKB:Q8N8S7"
}